{
  "term_id": "GO:0060336",
  "gene_name": "Protein mono-ADP-ribosyltransferase PARP14",
  "term_label": "negative regulation of type II interferon-mediated signaling pathway",
  "gene": "UniProtKB:Q460N5",
  "gene_symbol": "PARP14"
}